negative regulation of ATF6-mediated unfolded protein response [GO:1903892] (biological process) Definition: Any process that stops, prevents or reduces the frequency, rate or extent of the ATF6-mediated unfolded protein response. Also known as: down regulation of ATF6 branch of UPR, down regulation of ATF6-mediated unfolded protein response, down regulation of UPR signaling by ATF6 stress sensor, down regulation of activating transcription factor 6 signaling in unfolded protein response, down regulation of endoplasmic reticulum unfolded protein response; ATF6 signaling, down-regulation of ATF6 branch of UPR, down-regulation of ATF6-mediated unfolded protein response, down-regulation of UPR signaling by ATF6 stress sensor, down-regulation of activating transcription factor 6 signaling in unfolded protein response, down-regulation of endoplasmic reticulum unfolded protein response; ATF6 signaling, downregulation of ATF6 branch of UPR, downregulation of ATF6-mediated unfolded protein response, downregulation of UPR signaling by ATF6 stress sensor, downregulation of activating transcription factor 6 signaling in unfolded protein response, downregulation of endoplasmic reticulum unfolded protein response; ATF6 signaling, negative regulation of ATF6 branch of UPR, negative regulation of UPR signaling by ATF6 stress sensor, negative regulation of activating transcription factor 6 signaling in unfolded protein response, negative regulation of endoplasmic reticulum unfolded protein response; ATF6 signaling, down regulation of ATF6-alpha UPR branch, down regulation of ATF6-beta UPR branch, down-regulation of ATF6-alpha UPR branch, down-regulation of ATF6-beta UPR branch, downregulation of ATF6-alpha UPR branch, downregulation of ATF6-beta UPR branch, inhibition of ATF6 branch of UPR, inhibition of ATF6-alpha UPR branch, inhibition of ATF6-beta UPR branch, inhibition of ATF6-mediated unfolded protein response, inhibition of UPR signaling by ATF6 stress sensor, inhibition of activating transcription factor 6 signaling in unfolded protein response, inhibition of endoplasmic reticulum unfolded protein response; ATF6 signaling, negative regulation of ATF6-alpha UPR branch, negative regulation of ATF6-beta UPR branch, down regulation of ATF6 signaling in response to endoplasmic reticulum stress, down-regulation of ATF6 signaling in response to endoplasmic reticulum stress, downregulation of ATF6 signaling in response to endoplasmic reticulum stress, inhibition of ATF6 signaling in response to endoplasmic reticulum stress, negative regulation of ATF6 signaling in response to endoplasmic reticulum stress Relationships: is a type of negative regulation of endoplasmic reticulum unfolded protein response [GO:1900102]; is_a regulation of ATF6-mediated unfolded protein response [GO:1903891]; negatively regulates GO:0036500 References: PMID:22013210 Sources: GOC:PARL, GOC:TermGenie, GOC:bf, GO_REF:0000058